{
  "gene_symbol": "ZNF552",
  "term_label": "RNA polymerase II cis-regulatory region sequence-specific DNA binding",
  "gene": "UniProtKB:Q9H707",
  "gene_name": "Zinc finger protein 552",
  "term_id": "GO:0000978"
}